{
  "term_label": "cytoplasm",
  "term_id": "GO:0005737",
  "gene_name": "tRNA-dihydrouridine(20) synthase [NAD(P)+]-like",
  "gene_symbol": "DUS2",
  "gene": "UniProtKB:Q9NX74"
}